{
  "term_id": "GO:0005886",
  "term_label": "plasma membrane",
  "gene_symbol": "SLC26A6",
  "gene_name": "Solute carrier family 26 member 6",
  "gene": "UniProtKB:Q9BXS9"
}